t-UTP complex [GO:0034455] (cellular component) Relationships: is a type of nuclear protein-containing complex [GO:0140513]; is part of nucleolus [GO:0005730] Also known as: Nan1p-containing subcomplex of 90S preribosome References: PMID:17515605 Sources: GOC:krc, GOC:mah, GOC:vw Definition: A protein complex that forms a subcomplex of the 90S preribosome and is required for the subsequent assembly of the rest of the preribosome. In S. cerevisiae, it is composed of Utp5p, Utp4p, Nan1p, Utp8p, Utp9p, Utp10 and Utp15p. Note: Note that the term name uses Saccharomyces gene product names because no other names have yet arisen for this complex; the term nevertheless can be used for analogous complexes in other eukaryotes, and the name can be changed if better wording is found.